interleukin-1, type I, activating receptor activity [GO:0004909] (molecular function) References: PMID:15062641, PMID:18613828 Relationships: is a type of GO:0004908; is part of GO:0070498 Also known as: IL-1 type I, activating binding, IL-1 type I, activating receptor, interleukin-1 activating receptor activity, interleukin-1 type I receptor activity, interleukin-1, type I, activating binding Definition: Combining with interleukin-1 to initiate a change in cell activity via signaling pathways and mediated by adaptor proteins.